{
  "term_label": "adenylate cyclase-modulating G protein-coupled receptor signaling pathway",
  "gene": "UniProtKB:P41586",
  "gene_name": "Pituitary adenylate cyclase-activating polypeptide type I receptor",
  "term_id": "GO:0007188",
  "gene_symbol": "ADCYAP1R1"
}